{
  "gene_name": "Translation initiation factor eIF-2B subunit epsilon",
  "term_label": "guanyl-nucleotide exchange factor activity",
  "gene_symbol": "EIF2B5",
  "gene": "UniProtKB:Q13144",
  "term_id": "GO:0005085"
}